{
  "gene": "UniProtKB:P16233",
  "term_label": "triglyceride catabolic process",
  "gene_symbol": "PNLIP",
  "term_id": "GO:0019433",
  "gene_name": "Pancreatic triacylglycerol lipase"
}